{
  "term_id": "GO:0007165",
  "gene_symbol": "TTBK1",
  "gene": "UniProtKB:Q5TCY1",
  "gene_name": "Tau-tubulin kinase 1",
  "term_label": "signal transduction"
}